negative regulation of chromosome organization [GO:2001251] (biological process) Also known as: negative regulation of chromosome organisation, negative regulation of chromosome organization and biogenesis, negative regulation of maintenance of genome integrity, negative regulation of nuclear genome maintenance Definition: Any process that stops, prevents or reduces the frequency, rate or extent of chromosome organization. Relationships: is a type of negative regulation of organelle organization [GO:0010639]; is a type of regulation of chromosome organization [GO:0033044]; negatively regulates GO:0051276 Subtypes: negative regulation of telomere maintenance [GO:0032205], negative regulation of sister chromatid segregation [GO:0033046], GO:0045875, negative regulation of oocyte karyosome formation [GO:0120314], negative regulation of chromosome condensation [GO:1902340], negative regulation of kinetochore assembly [GO:1905560] Sources: GOC:obol